{
  "gene": "UniProtKB:O14770",
  "term_label": "nucleus",
  "gene_name": "Homeobox protein Meis2",
  "gene_symbol": "MEIS2",
  "term_id": "GO:0005634"
}